{
  "gene": "UniProtKB:Q9HB21",
  "gene_symbol": "PLEKHA1",
  "term_id": "GO:0051898",
  "term_label": "negative regulation of phosphatidylinositol 3-kinase/protein kinase B signal transduction",
  "gene_name": "Pleckstrin homology domain-containing family A member 1"
}